{
  "term_id": "UNKNOWN:0003",
  "gene": "UniProtKB:Q5XKK7",
  "term_label": "Unknown cellular component",
  "gene_symbol": "FAM219B",
  "gene_name": "Protein FAM219B"
}